{
  "gene_symbol": "PELI3",
  "gene": "UniProtKB:Q8N2H9",
  "term_label": "ubiquitin protein ligase activity",
  "gene_name": "E3 ubiquitin-protein ligase pellino homolog 3",
  "term_id": "GO:0061630"
}